collateral sprouting of injured axon [GO:0048674] (biological process) Sources: GOC:dgh, GOC:dph, GOC:jid, GOC:lm Relationships: is a type of collateral sprouting [GO:0048668]; is a type of sprouting of injured axon [GO:0048682] Regulation: regulated by GO:0048693; positively regulated by positive regulation of collateral sprouting of injured axon [GO:0048694]; negatively regulated by negative regulation of collateral sprouting of injured axon [GO:0048695] Definition: The process resulting in reformation of a growth cone by the tip of an injured axon, or in collateral sprouting of the axon. Collateral sprouting is the process in which outgrowths develop from the shafts of existing axons.